{
  "term_id": "UNKNOWN:0001",
  "gene_name": "Leucine-rich repeat-containing protein 43",
  "term_label": "Unknown molecular function",
  "gene_symbol": "LRRC43",
  "gene": "UniProtKB:Q8N309"
}